{
  "term_id": "GO:0097401",
  "gene_name": "V-type proton ATPase subunit G 3",
  "gene_symbol": "ATP6V1G3",
  "gene": "UniProtKB:Q96LB4",
  "term_label": "synaptic vesicle lumen acidification"
}